{
  "gene_name": "Trifunctional purine biosynthetic protein adenosine-3",
  "gene": "UniProtKB:P22102",
  "term_label": "phosphoribosylamine-glycine ligase activity",
  "term_id": "GO:0004637",
  "gene_symbol": "GART"
}